{
  "gene": "UniProtKB:P58753",
  "gene_name": "Toll_interleukin-1 receptor domain-containing adapter protein",
  "term_label": "Toll-like receptor 4 binding",
  "gene_symbol": "TIRAP",
  "term_id": "GO:0035662"
}